{
  "gene_symbol": "CACNG2",
  "gene": "UniProtKB:Q9Y698",
  "term_id": "GO:0098839",
  "gene_name": "Voltage-dependent calcium channel gamma-2 subunit",
  "term_label": "postsynaptic density membrane"
}